energy coupled proton transmembrane transport, against electrochemical gradient [GO:0015988] (biological process) Sources: GOC:mah Subtypes: electron transport coupled proton transport [GO:0015990] Definition: The transport of protons across a membrane and against an electrochemical gradient, using energy from a source such as ATP hydrolysis, light, or electron transport. Relationships: is a type of proton transmembrane transport [GO:1902600]